galactoglucomannan metabolic process [GO:0010392] (biological process) Definition: The chemical reactions and pathways involving galactoglucomannan, a polysaccharide composed of D-glucose, D-galactose and D-mannose. The mannose units form the backbone structure (a linear main chain) decorated with a mixture of D-glucose and D-galactose side-units. Sources: GOC:tair_curators Subtypes: galactoglucomannan catabolic process [GO:2000885] Relationships: is a type of substituted mannan metabolic process [GO:0006080] Also known as: galactoglucomannan metabolism